nickel incorporation into iron-sulfur cluster via tris-L-cysteinyl L-cysteine persulfido L-glutamato L-histidino L-serinyl nickel triiron disulfide trioxide [GO:0018418] (biological process) Definition: The incorporation of nickel into a 3Fe-2S complex by tris-L-cysteinyl L-cysteine persulfido L-glutamato L-histidino L-serinyl nickel triiron disulfide trioxide. Also known as: nickel incorporation into iron-sulphur cluster via tris-L-cysteinyl L-cysteine persulphido L-glutamato L-histidino L-serinyl nickel triiron disulphide trioxide Sources: RESID:AA0293 Relationships: is a type of iron-sulfur cluster assembly [GO:0016226]; is a type of peptidyl-cysteine modification [GO:0018198]; is_a peptidyl-glutamic acid modification [GO:0018200]; is a type of peptidyl-histidine modification [GO:0018202]; is a type of nickel incorporation into metallo-sulfur cluster [GO:0018414]